{
  "term_label": "serine-type endopeptidase activity",
  "gene_name": "Kallikrein-14",
  "term_id": "GO:0004252",
  "gene_symbol": "KLK14",
  "gene": "UniProtKB:Q9P0G3"
}